{
  "term_label": "glucuronosyltransferase activity",
  "gene": "UniProtKB:P54855",
  "gene_symbol": "UGT2B15",
  "term_id": "GO:0015020",
  "gene_name": "UDP-glucuronosyltransferase 2B15"
}